{
  "term_id": "GO:0000981",
  "gene_symbol": "TEF",
  "gene_name": "Thyrotroph embryonic factor",
  "term_label": "DNA-binding transcription factor activity, RNA polymerase II-specific",
  "gene": "UniProtKB:Q10587"
}